{
  "gene_name": "Ankyrin repeat domain-containing protein 23",
  "term_label": "positive regulation of transcription by RNA polymerase II",
  "gene_symbol": "ANKRD23",
  "term_id": "GO:0045944",
  "gene": "UniProtKB:Q86SG2"
}